negative regulation of T cell costimulation [GO:2000524] (biological process) Also known as: negative regulation of T cell co-stimulation, negative regulation of T lymphocyte costimulation, negative regulation of T-cell co-stimulation, negative regulation of T-cell costimulation, negative regulation of T-lymphocyte costimulation Subtypes: negative regulation of CD4-positive, alpha-beta T cell costimulation [GO:1900280] Definition: Any process that stops, prevents or reduces the frequency, rate or extent of T cell costimulation. Relationships: is_a negative regulation of immune system process [GO:0002683]; is a type of GO:2000523; negatively regulates T cell costimulation [GO:0031295] Sources: GOC:obol